{
  "gene_symbol": "IFT88",
  "term_id": "GO:0097546",
  "gene_name": "Intraflagellar transport protein 88 homolog",
  "gene": "UniProtKB:Q13099",
  "term_label": "ciliary base"
}